{
  "gene_name": "Cytochrome P450 2C19",
  "term_id": "GO:0042178",
  "gene": "UniProtKB:P33261",
  "term_label": "xenobiotic catabolic process",
  "gene_symbol": "CYP2C19"
}